{
  "term_label": "smoothened signaling pathway",
  "term_id": "GO:0007224",
  "gene": "UniProtKB:Q96GX1",
  "gene_symbol": "TCTN2",
  "gene_name": "Tectonic-2"
}